{
  "gene": "UniProtKB:Q14397",
  "gene_name": "Glucokinase regulatory protein",
  "term_id": "GO:0005654",
  "term_label": "nucleoplasm",
  "gene_symbol": "GCKR"
}